{
  "gene": "UniProtKB:P54317",
  "gene_name": "Pancreatic lipase-related protein 2",
  "term_id": "GO:0009395",
  "term_label": "phospholipid catabolic process",
  "gene_symbol": "PNLIPRP2"
}